response to iron ion [GO:0010039] (BP) Relationships: is a type of response to metal ion [GO:0010038] Also known as: response to iron Subtypes: response to iron(II) ion [GO:0010040], response to iron(III) ion [GO:0010041], cellular response to iron ion [GO:0071281] Definition: Any process that results in a change in state or activity of a cell or an organism (in terms of movement, secretion, enzyme production, gene expression, etc.) as a result of an iron ion stimulus. Sources: GOC:sm